{
  "gene": "UniProtKB:Q8TAT5",
  "term_id": "GO:0005634",
  "gene_name": "Endonuclease 8-like 3",
  "term_label": "nucleus",
  "gene_symbol": "NEIL3"
}